mesenchymal cell proliferation involved in ureteric bud development [GO:0072138] (biological process) Sources: GOC:mtg_kidney_jan10 Definition: The multiplication or reproduction of cells, resulting in the expansion of a mesenchymal cell population of the ureteric bud, that contributes to ureteric bud development. Also known as: ureteric bud mesenchymal cell proliferation Relationships: is a type of GO:0010463; is a type of GO:0061209; BFO_0000050 GO:0001657